{
  "gene": "UniProtKB:Q6PEX7",
  "term_id": "UNKNOWN:0001",
  "gene_symbol": "TEX38",
  "gene_name": "Testis-expressed protein 38",
  "term_label": "Unknown molecular function"
}